{
  "gene_symbol": "HPRT1",
  "gene_name": "Hypoxanthine-guanine phosphoribosyltransferase",
  "term_id": "GO:0004422",
  "term_label": "hypoxanthine phosphoribosyltransferase activity",
  "gene": "UniProtKB:P00492"
}